{
  "term_label": "cytokine activity",
  "gene_name": "Proto-oncogene Wnt-1",
  "gene_symbol": "WNT1",
  "term_id": "GO:0005125",
  "gene": "UniProtKB:P04628"
}